{
  "gene": "UniProtKB:Q8TDX5",
  "gene_name": "2-amino-3-carboxymuconate-6-semialdehyde decarboxylase",
  "term_id": "GO:0005737",
  "gene_symbol": "ACMSD",
  "term_label": "cytoplasm"
}